{
  "term_label": "plasma membrane",
  "gene_name": "Phosphatidylinositol 4-phosphate 5-kinase type-1 alpha",
  "term_id": "GO:0005886",
  "gene_symbol": "PIP5K1A",
  "gene": "UniProtKB:Q99755"
}